3-hydroxyphenylpropionic acid transmembrane transporter activity [GO:0042926] (molecular function) Relationships: is a type of monocarboxylic acid transmembrane transporter activity [GO:0008028]; is a type of xenobiotic transmembrane transporter activity [GO:0042910]; is part of GO:0042920 Also known as: 3-(3-hydroxyphenyl)propionic acid transporter activity, m-hydroxyphenylpropionic acid transporter activity, 3-hydroxyphenylpropionic acid transporter activity References: PMID:9098055 Sources: GOC:jl Definition: Enables the directed movement of 3-hydroxyphenylpropionic acid from one side of a membrane to the other.